steroid dehydrogenase activity [GO:0016229] (molecular function) Definition: Catalysis of an oxidation-reduction (redox) reaction in which one substrate is a sterol derivative. Relationships: is a type of GO:0016491 Sources: GOC:mah Subtypes: GO:0033764, steroid dehydrogenase activity, acting on the CH-CH group of donors [GO:0033765]